{
  "gene_symbol": "GATD3B",
  "gene_name": "Putative glutamine amidotransferase-like class 1 domain-containing protein 3B, mitochondrial",
  "gene": "UniProtKB:A0A0B4J2D5",
  "term_label": "Unknown molecular function",
  "term_id": "UNKNOWN:0001"
}